{
  "gene_name": "NPC intracellular cholesterol transporter 1",
  "gene": "UniProtKB:O15118",
  "gene_symbol": "NPC1",
  "term_id": "GO:0015918",
  "term_label": "sterol transport"
}